{
  "term_label": "microtubule associated complex",
  "term_id": "GO:0005875",
  "gene": "UniProtKB:O95239",
  "gene_symbol": "KIF4A",
  "gene_name": "Chromosome-associated kinesin KIF4A"
}